regulation of rRNA processing [GO:2000232] (biological process) Subtypes: GO:2000233, GO:2000234 Definition: Any process that modulates the frequency, rate or extent of rRNA processing. Also known as: regulation of 35S primary transcript processing Sources: GOC:mah Relationships: is a type of regulation of gene expression [GO:0010468]; is a type of GO:0051252; regulates rRNA processing [GO:0006364]